protein localization to ascospore wall [GO:1904853] (biological process) Also known as: protein localisation in ascospore wall, protein localisation to ascospore wall, protein localization in ascospore wall Relationships: is a type of protein localization to spore cell wall [GO:0099614] Definition: A process in which a protein is transported to, or maintained in, a location within an ascospore wall. References: PMID:24623719 Sources: GOC:TermGenie, GO_REF:0000087